{
  "gene": "UniProtKB:Q13188",
  "term_id": "GO:0043408",
  "term_label": "regulation of MAPK cascade",
  "gene_symbol": "STK3",
  "gene_name": "Serine_threonine-protein kinase 3"
}